{
  "gene_name": "Cyclin-Y-like protein 1",
  "term_label": "cyclin-dependent protein serine/threonine kinase activator activity",
  "gene_symbol": "CCNYL1",
  "term_id": "GO:0061575",
  "gene": "UniProtKB:Q8N7R7"
}